ERAD pathway [GO:0036503] (biological process) Relationships: is a type of proteasomal protein catabolic process [GO:0010498]; is a type of response to endoplasmic reticulum stress [GO:0034976]; is a type of response to nitrogen compound [GO:1901698] Also known as: endoplasmic reticulum-associated degradation, protein degradation by ERAD, ER-associated degradation pathway, endoplasmic reticulum-associated protein degradation pathway Subtypes: ubiquitin-dependent glycoprotein ERAD pathway [GO:0097466] References: PMID:20940304, PMID:21969857 Sources: GOC:PARL, GOC:bf Regulation: regulated by GO:1904292; negatively regulated by GO:1904293; positively regulated by positive regulation of ERAD pathway [GO:1904294] Definition: The protein catabolic pathway which targets endoplasmic reticulum (ER)-resident proteins for degradation by the cytoplasmic proteasome. It begins with recognition of the ER-resident protein, includes retrotranslocation (dislocation) of the protein from the ER to the cytosol, protein modifications necessary for correct substrate transfer (e.g. ubiquitination), transport of the protein to the proteasome, and ends with degradation of the protein by the cytoplasmic proteasome. Note: ER-associated protein degradation (ERAD) pathways target misfolded ER lumenal proteins (ERAD-L), ER membrane proteins (ERAD-M), and ER proteins with misfolded cytosolic domains (ERAD-C) by recognizing aberrant proteins, retrotranslocating these substrates to the cytosol, followed by substrate ubiquitination and proteosomal-mediated degradation. In contrast the stress-induced homeostatically regulated protein degradation (SHRED) pathway (GO:0120174), although inducible by stress, targets diverse ER membrane, and cytosolic proteins as well as numerous other native proteins in the absence of stress. Stress results in the protease-mediated (Nma111p) generation of a Roq1p cleavage product that then binds to the type-1 active site of Ubr1p, altering its substrate specificity, and leading to the proteasome-mediated degradation of both misfolded and native proteins. Although the SHRED pathway may contain some components in common with ERAD pathways (GO:0036503), such as UBR1, RAD6 and CDC48, other ERAD components, such as HRD1 and DOA10, do not appear to be involved, and as such these pathways are currently considered to be distinct.